{
  "term_label": "cytosol",
  "term_id": "GO:0005829",
  "gene_symbol": "MAP3K20",
  "gene": "UniProtKB:Q9NYL2",
  "gene_name": "Mitogen-activated protein kinase kinase kinase 20"
}